{
  "term_label": "Unknown biological process",
  "gene_symbol": "KRTAP11-1",
  "gene_name": "Keratin-associated protein 11-1",
  "gene": "UniProtKB:Q8IUC1",
  "term_id": "UNKNOWN:0002"
}